{
  "term_id": "GO:0005829",
  "gene": "UniProtKB:P56537",
  "gene_name": "Eukaryotic translation initiation factor 6",
  "gene_symbol": "EIF6",
  "term_label": "cytosol"
}